13-hydroxydocosanoate 13-beta-glucosyltransferase activity [GO:0047229] (molecular function) Sources: EC:2.4.1.158 Relationships: is a type of UDP-glucosyltransferase activity [GO:0035251] Definition: Catalysis of the reaction: 13-hydroxydocosanoate + UDP-D-glucose = 13-beta-D-glucosyloxydocosanoate + UDP. Also known as: 13-glucosyloxydocosanoate 2'-beta-glucosyltransferase activity, UDP-glucose-13-hydroxydocosanoate glucosyltransferase activity, UDP-glucose:13-hydroxydocosanoate 13-beta-D-glucosyltransferase activity, UDP-glucose:13-hydroxydocosanoic acid glucosyltransferase activity, UDPglucose:13-hydroxydocosanoate 13-beta-D-glucosyltransferase activity, uridine diphosphoglucose-hydroxydocosanoate glucosyltransferase activity